{
  "term_label": "UDP-galactose transmembrane transporter activity",
  "gene": "UniProtKB:P78383",
  "term_id": "GO:0005459",
  "gene_symbol": "SLC35B1",
  "gene_name": "Solute carrier family 35 member B1"
}